{
  "term_label": "negative regulation of complement activation, classical pathway",
  "gene": "UniProtKB:P17927",
  "term_id": "GO:0045959",
  "gene_name": "Complement receptor type 1",
  "gene_symbol": "CR1"
}